{
  "term_id": "GO:0003735",
  "gene": "UniProtKB:P62851",
  "term_label": "structural constituent of ribosome",
  "gene_name": "Small ribosomal subunit protein eS25",
  "gene_symbol": "RPS25"
}